regulation of DNA replication termination [GO:2000621] (biological process) Subtypes: GO:0097046 Sources: GOC:obol Definition: Any process that modulates the frequency, rate or extent of DNA replication termination. Relationships: is a type of regulation of DNA-templated DNA replication [GO:0090329]; regulates DNA replication termination [GO:0006274]